{
  "gene_name": "Globoside alpha-1,3-N-acetylgalactosaminyltransferase 1",
  "gene": "UniProtKB:Q8N5D6",
  "term_id": "GO:0005794",
  "term_label": "Golgi apparatus",
  "gene_symbol": "GBGT1"
}